{
  "gene_symbol": "BCOR",
  "gene": "UniProtKB:Q6W2J9",
  "gene_name": "BCL-6 corepressor",
  "term_id": "GO:0005634",
  "term_label": "nucleus"
}